{
  "gene_name": "Small membrane A-kinase anchor protein",
  "term_label": "Unknown cellular component",
  "gene_symbol": "C2orf88",
  "term_id": "UNKNOWN:0003",
  "gene": "UniProtKB:Q9BSF0"
}